{
  "gene": "UniProtKB:Q92621",
  "gene_symbol": "NUP205",
  "term_id": "GO:0006999",
  "term_label": "nuclear pore organization",
  "gene_name": "Nuclear pore complex protein Nup205"
}